vesicle tethering involved in exocytosis [GO:0090522] (biological process) Subtypes: GO:0098881, GO:0099069, contractile vacuole tethering involved in discharge [GO:0140025] References: PMID:10559876, PMID:17052174, PMID:17488620, PMID:22420621, PMID:27243008 Sources: GOC:rn Definition: The initial, indirect interaction between a secretory vesicle membrane and a site of exocytosis in the plasma membrane. This interaction is mediated by tethering factors (or complexes), which interact with both membranes. Interaction can occur via direct binding to membrane phospholipids or membrane proteins, or via binding to vesicle coat proteins. This process is distinct from and prior to docking and fusion. Relationships: is a type of GO:0099022; is_a exocytic process [GO:0140029] Also known as: vesicle tethering to plasma membrane